{
  "gene_symbol": "LCE3D",
  "term_id": "UNKNOWN:0003",
  "term_label": "Unknown cellular component",
  "gene_name": "Late cornified envelope protein 3D",
  "gene": "UniProtKB:Q9BYE3"
}